{
  "gene_name": "Voltage-dependent L-type calcium channel subunit beta-4",
  "term_label": "chemical synaptic transmission",
  "gene": "UniProtKB:O00305",
  "term_id": "GO:0007268",
  "gene_symbol": "CACNB4"
}